{
  "gene_symbol": "VPS72",
  "term_label": "chromatin remodeling",
  "gene": "UniProtKB:Q15906",
  "term_id": "GO:0006338",
  "gene_name": "Vacuolar protein sorting-associated protein 72 homolog"
}